{
  "gene": "UniProtKB:A0A075B6H9",
  "gene_name": "Immunoglobulin lambda variable 4-69",
  "term_label": "immune response",
  "term_id": "GO:0006955",
  "gene_symbol": "IGLV4-69"
}